{
  "term_id": "GO:0003906",
  "gene": "UniProtKB:Q96FI4",
  "term_label": "DNA-(apurinic or apyrimidinic site) endonuclease activity",
  "gene_symbol": "NEIL1",
  "gene_name": "Endonuclease 8-like 1"
}